{
  "term_id": "GO:0070740",
  "gene_symbol": "TTLL11",
  "gene": "UniProtKB:Q8NHH1",
  "gene_name": "Tubulin polyglutamylase TTLL11",
  "term_label": "tubulin-glutamic acid ligase activity"
}